poly-ADP-D-ribose modification-dependent protein binding [GO:0160004] (molecular function) References: PMID:26673700 Definition: Binding to a protein upon poly-ADP-ribosylation of the target protein. Note: This term should only be used when the binding is shown to require a poly-ADP-D-ribose post-translational modification: the interaction needs to be tested with and without the PTM. The binding does not need to be at the site of the ADP-D-ribose modification. It may be that the PTM causes a conformational change that allows binding of the protein to another region; this type of modification-dependent protein binding is valid for annotation to this term. Relationships: is a type of ADP-D-ribose modification-dependent protein binding [GO:0160002]